pyridoxine 4-dehydrogenase (NADP+) activity [GO:0050236] (molecular function) Relationships: is a type of GO:0008106 Sources: RHEA:16129 Definition: Catalysis of the reaction: NADP+ + pyridoxine = H+ + NADPH + pyridoxal. Also known as: pyridoxine:NADP 4-dehydrogenase activity, PL reductase activity, pyridoxal reductase activity, pyridoxin dehydrogenase activity, pyridoxine dehydrogenase activity, pyridoxine:NADP 4-oxidoreductase activity, pyridoxol dehydrogenase activity